{
  "gene_name": "Receptor activity-modifying protein 1",
  "gene_symbol": "RAMP1",
  "gene": "UniProtKB:O60894",
  "term_id": "GO:0031623",
  "term_label": "receptor internalization"
}